{
  "term_id": "GO:0004364",
  "gene_symbol": "GSTA4",
  "gene_name": "Glutathione S-transferase A4",
  "term_label": "glutathione transferase activity",
  "gene": "UniProtKB:O15217"
}